{
  "gene_symbol": "POTEI",
  "term_id": "GO:0048870",
  "gene_name": "POTE ankyrin domain family member I",
  "term_label": "cell motility",
  "gene": "UniProtKB:P0CG38"
}